cytokinin binding [GO:0044373] (molecular function) Definition: Binding to a cytokinin, any of a class of adenine-derived compounds that can function in plants as growth regulators. Sources: GOC:jl Relationships: is a type of hormone binding [GO:0042562]